{
  "term_label": "chemoattractant activity",
  "gene_name": "Secretogranin-2",
  "gene": "UniProtKB:P13521",
  "gene_symbol": "SCG2",
  "term_id": "GO:0042056"
}